trophectodermal cellular morphogenesis [GO:0001831] (biological process) Note: See also the Anatomical Dictionary for Mouse Development ontology terms 'TS4, trophectoderm ; EMAP:19', 'TS5, trophectoderm ; EMAP:28' and 'TS6, trophectoderm ; EMAP:39'. Definition: The morphogenesis of trophectoderm cells. Relationships: is a type of cell morphogenesis [GO:0000902]; is a type of GO:0048598; is part of trophectodermal cell differentiation [GO:0001829] Sources: GOC:dph, ISBN:0124020607, ISBN:0198542771 Also known as: trophectoderm cellular morphogenesis